negative regulation of smoothened signaling pathway [GO:0045879] (biological process) Subtypes: negative regulation of smoothened signaling pathway involved in ventral spinal cord patterning [GO:0021914], negative regulation of smoothened signaling pathway involved in dorsal/ventral neural tube patterning [GO:1901621], negative regulation of hh target transcription factor activity [GO:1990787] Relationships: is a type of GO:0008589; is a type of negative regulation of signal transduction [GO:0009968]; negatively regulates smoothened signaling pathway [GO:0007224] Also known as: down regulation of smoothened signaling pathway, down-regulation of smoothened signaling pathway, downregulation of smoothened signaling pathway, negative regulation of hedgehog signaling pathway, negative regulation of hh signaling pathway, negative regulation of smoothened signalling pathway, inhibition of smoothened signaling pathway, negative regulation of smoothened by patched, negative regulation of smoothened activity, negative regulation of smoothened receptor activity by patched Definition: Any process that stops, prevents, or reduces the frequency, rate or extent of smoothened signaling. Sources: GOC:go_curators